{
  "term_label": "positive regulation of TOR signaling",
  "gene_name": "Protein SEC13 homolog",
  "gene_symbol": "SEC13",
  "term_id": "GO:0032008",
  "gene": "UniProtKB:P55735"
}